{
  "term_id": "GO:0005634",
  "gene_symbol": "NSMCE4A",
  "term_label": "nucleus",
  "gene": "UniProtKB:Q9NXX6",
  "gene_name": "Non-structural maintenance of chromosomes element 4 homolog A"
}